{
  "term_id": "GO:0012506",
  "gene_name": "Annexin A2",
  "term_label": "vesicle membrane",
  "gene": "UniProtKB:P07355",
  "gene_symbol": "ANXA2"
}